{
  "gene": "UniProtKB:Q9Y4F9",
  "gene_name": "Rho family-interacting cell polarization regulator 2",
  "term_label": "Unknown biological process",
  "term_id": "UNKNOWN:0002",
  "gene_symbol": "RIPOR2"
}